{
  "term_label": "Unknown cellular component",
  "gene_name": "Janus kinase and microtubule-interacting protein 1",
  "gene": "UniProtKB:Q96N16",
  "term_id": "UNKNOWN:0003",
  "gene_symbol": "JAKMIP1"
}